{
  "term_label": "transforming growth factor beta receptor activity, type I",
  "gene_name": "TGF-beta receptor type-1",
  "term_id": "GO:0005025",
  "gene": "UniProtKB:P36897",
  "gene_symbol": "TGFBR1"
}